B cell proliferation involved in immune response [GO:0002322] (biological process) Sources: GOC:jal Also known as: B cell proliferation during immune response, B lymphocyte proliferation during immune response, B-cell proliferation during immune response, B-lymphocyte proliferation during immune response Relationships: is a type of B cell activation involved in immune response [GO:0002312]; is a type of B cell proliferation [GO:0042100] Definition: The expansion of a B cell population by cell division following B cell activation during an immune response.